{
  "term_label": "nucleus",
  "gene_name": "Zinc finger protein 177",
  "gene": "UniProtKB:Q13360",
  "gene_symbol": "ZNF177",
  "term_id": "GO:0005634"
}